{
  "gene_symbol": "PAQR5",
  "gene_name": "Membrane progestin receptor gamma",
  "term_label": "signaling receptor activity",
  "gene": "UniProtKB:Q9NXK6",
  "term_id": "GO:0038023"
}